{
  "term_label": "Unknown biological process",
  "gene": "UniProtKB:Q5TZK3",
  "gene_symbol": "FAM74A6",
  "gene_name": "Protein FAM74A4_A6",
  "term_id": "UNKNOWN:0002"
}